{
  "term_id": "GO:0006511",
  "gene": "UniProtKB:O95376",
  "term_label": "ubiquitin-dependent protein catabolic process",
  "gene_name": "E3 ubiquitin-protein ligase ARIH2",
  "gene_symbol": "ARIH2"
}